{
  "gene_name": "TBC domain-containing protein kinase-like protein",
  "gene": "UniProtKB:Q8TEA7",
  "term_id": "UNKNOWN:0003",
  "term_label": "Unknown cellular component",
  "gene_symbol": "TBCK"
}